{
  "gene_name": "Ropporin-1B",
  "gene_symbol": "ROPN1B",
  "term_id": "GO:0048240",
  "term_label": "sperm capacitation",
  "gene": "UniProtKB:Q9BZX4"
}